{
  "gene_name": "T cell receptor beta variable 6-2",
  "gene": "UniProtKB:A0A0J9YXY3",
  "term_id": "GO:0007166",
  "term_label": "cell surface receptor signaling pathway",
  "gene_symbol": "TRBV6-2"
}